{
  "term_id": "GO:0005783",
  "gene_name": "Mannosyl-oligosaccharide 1,2-alpha-mannosidase IA",
  "term_label": "endoplasmic reticulum",
  "gene_symbol": "MAN1A1",
  "gene": "UniProtKB:P33908"
}